{
  "gene_symbol": "ANGPT4",
  "term_id": "GO:0031012",
  "gene_name": "Angiopoietin-4",
  "term_label": "extracellular matrix",
  "gene": "UniProtKB:Q9Y264"
}